{
  "gene_symbol": "B3GAT3",
  "gene_name": "Galactosylgalactosylxylosylprotein 3-beta-glucuronosyltransferase 3",
  "term_label": "galactosylgalactosylxylosylprotein 3-beta-glucuronosyltransferase activity",
  "term_id": "GO:0015018",
  "gene": "UniProtKB:O94766"
}